apolipoprotein binding [GO:0034185] (molecular function) Definition: Binding to an apolipoprotein, the protein component of a lipoprotein complex. Subtypes: apolipoprotein A-I binding [GO:0034186] Relationships: is a type of protein binding [GO:0005515] Sources: GOC:BHF, GOC:rl